{
  "term_label": "cytosol",
  "gene": "UniProtKB:Q14568",
  "term_id": "GO:0005829",
  "gene_symbol": "HSP90AA2P",
  "gene_name": "Heat shock protein HSP 90-alpha A2"
}